{
  "gene_name": "Protocadherin alpha-C1",
  "term_id": "GO:0050839",
  "gene": "UniProtKB:Q9H158",
  "gene_symbol": "PCDHAC1",
  "term_label": "cell adhesion molecule binding"
}